{
  "term_label": "lysosomal membrane",
  "gene_name": "Putative uncharacterized protein SLC66A1L",
  "term_id": "GO:0005765",
  "gene_symbol": "SLC66A1LP",
  "gene": "UniProtKB:A1A4F0"
}